{
  "gene_symbol": "APOA5",
  "gene": "UniProtKB:Q6Q788",
  "term_label": "cholesterol metabolic process",
  "gene_name": "Apolipoprotein A-V",
  "term_id": "GO:0008203"
}